phosphodiesterase activity, acting on 3'-phosphoglycolate-terminated DNA strands [GO:0090580] (molecular function) Definition: Catalysis of the hydrolytic removal of phosphoglycolate from the 3'-terminus of a 3'-phosphoglycolate-terminated DNA strand. References: PMID:11238902 Sources: GOC:pde, GOC:rb Relationships: is a type of phosphoric diester hydrolase activity [GO:0008081]; is a type of catalytic activity, acting on DNA [GO:0140097]